{
  "term_id": "UNKNOWN:0002",
  "gene_symbol": "CA5B",
  "gene": "UniProtKB:Q9Y2D0",
  "term_label": "Unknown biological process",
  "gene_name": "Carbonic anhydrase 5B, mitochondrial"
}